{
  "gene": "UniProtKB:Q4LDE5",
  "term_label": "Unknown cellular component",
  "gene_symbol": "SVEP1",
  "term_id": "UNKNOWN:0003",
  "gene_name": "Sushi, von Willebrand factor type A, EGF and pentraxin domain-containing protein 1"
}